{
  "gene_name": "IQ motif and SEC7 domain-containing protein 2",
  "term_id": "GO:0098839",
  "term_label": "postsynaptic density membrane",
  "gene_symbol": "IQSEC2",
  "gene": "UniProtKB:Q5JU85"
}